{
  "term_id": "GO:0002456",
  "gene_name": "Complement receptor type 1",
  "term_label": "T cell mediated immunity",
  "gene_symbol": "CR1",
  "gene": "UniProtKB:P17927"
}